{
  "gene_symbol": "TRIM38",
  "term_id": "GO:0005737",
  "gene": "UniProtKB:O00635",
  "term_label": "cytoplasm",
  "gene_name": "E3 ubiquitin-protein ligase TRIM38"
}